{
  "term_label": "Unknown biological process",
  "gene_name": "Uncharacterized protein C3orf62",
  "term_id": "UNKNOWN:0002",
  "gene": "UniProtKB:Q6ZUJ4",
  "gene_symbol": "C3orf62"
}